methylenetetrahydromethanopterin dehydrogenase activity [GO:0030268] (molecular function) Also known as: 5,10-methylenetetrahydromethanopterin dehydrogenase activity, 5,10-methylenetetrahydromethanopterin:coenzyme-F420 oxidoreductase activity, N(5),N(10)-methylenetetrahydromethanopterin dehydrogenase activity Sources: EC:1.5.98.1, RHEA:16721 Relationships: is a type of GO:0016645 Definition: Catalysis of the reaction: 5,10-methylenetetrahydromethanopterin + coenzyme F420 + 2 H+ = 5,10-methenyl-5,6,7,8-tetrahydromethanopterin + reduced coenzyme F420.